symbiont-mediated activation of host interferon signaling pathway [GO:0141080] (biological process) Definition: A process in which a symbiont subverts an interferon-mediated signal transduction pathway in the host organism by initiating, promoting, or enhancing its activation. References: PMID:26553469, PMID:29076073 Relationships: is a type of symbiont-mediated activation of host signal transduction pathway [GO:0052028]